{
  "gene_symbol": "ADA",
  "term_id": "GO:0042110",
  "gene_name": "Adenosine deaminase",
  "term_label": "T cell activation",
  "gene": "UniProtKB:P00813"
}